{
  "gene": "UniProtKB:O75391",
  "gene_name": "Sperm-associated antigen 7",
  "term_label": "Unknown biological process",
  "term_id": "UNKNOWN:0002",
  "gene_symbol": "SPAG7"
}